{
  "gene_symbol": "RFPL2",
  "term_id": "GO:0010468",
  "gene": "UniProtKB:O75678",
  "gene_name": "Ret finger protein-like 2",
  "term_label": "regulation of gene expression"
}